{
  "term_label": "histone deacetylase complex",
  "gene_symbol": "KDM3A",
  "gene": "UniProtKB:Q9Y4C1",
  "term_id": "GO:0000118",
  "gene_name": "Lysine-specific demethylase 3A"
}